{
  "gene": "UniProtKB:Q15834",
  "gene_name": "Coiled-coil domain-containing protein 85B",
  "term_label": "Unknown molecular function",
  "term_id": "UNKNOWN:0001",
  "gene_symbol": "CCDC85B"
}